auditory receptor cell development [GO:0060117] (BP) Sources: GOC:dph Definition: The process whose specific outcome is the progression of an auditory receptor cell over time, from its formation to the mature structure. Cell development does not include the steps involved in committing a cell to a specific fate. Relationships: is a type of inner ear receptor cell development [GO:0060119]; BFO_0000050 inner ear auditory receptor cell differentiation [GO:0042491] Also known as: auditory hair cell development